negative regulation of mast cell apoptotic process [GO:0033026] (biological process) Relationships: is a type of negative regulation of immune system process [GO:0002683]; is a type of regulation of mast cell apoptotic process [GO:0033025]; is a type of negative regulation of myeloid cell apoptotic process [GO:0033033]; is a type of GO:2000107; negatively regulates mast cell apoptotic process [GO:0033024] Also known as: down regulation of mast cell apoptosis, down-regulation of mast cell apoptosis, downregulation of mast cell apoptosis, inhibition of mast cell apoptosis, negative regulation of mast cell apoptosis Sources: GOC:add, GOC:mtg_apoptosis Definition: Any process that stops, prevents, or reduces the frequency, rate, or extent of mast cell apoptotic process.